regulation of axo-dendritic protein transport [GO:1905126] (biological process) Also known as: regulation of axonal protein transport Relationships: is a type of regulation of intracellular protein transport [GO:0033157]; is a type of GO:0060632; regulates axo-dendritic protein transport [GO:0099640] Subtypes: GO:1905127, GO:1905128 References: PMID:20694152 Sources: GOC:TermGenie, GO_REF:0000058 Definition: Any process that modulates the frequency, rate or extent of axo-dendritic protein transport.